cell rearrangement involved in Malpighian tubule morphogenesis [GO:0061334] (biological process) Sources: GOC:dph, GOC:mtg_kidney_jan10 Relationships: is a type of cell migration [GO:0016477]; is part of Malpighian tubule morphogenesis [GO:0007443] Also known as: cell migration involved in Malpighian tubule morphogenesis Subtypes: GO:0061352 Definition: The movement of an epithelial cell with respect to other epithelial cells that contributes to the shaping of the Malpighian tubule.